sinapoylglucose-sinapoylglucose O-sinapoyltransferase activity [GO:0047158] (molecular function) Also known as: 1-(hydroxycinnamoyl)-glucose:1-(hydroxycinnamoyl)-glucose hydroxycinnamoyltransferase activity, 1-O-(4-hydroxy-3,5-dimethoxycinnamoyl)-beta-D-glucoside:1-O-(4-hydroxy-3,5-dimethoxycinnamoyl-beta-D-glucoside 1-O-sinapoyltransferase activity, hydroxycinnamoylglucose-hydroxycinnamoylglucose hydroxycinnamoyltransferase activity Definition: Catalysis of the reaction: 2 1-O-sinapoyl-beta-D-glucose = 1,2-di-O-sinapoyl-beta-D-glucose + D-glucose. Relationships: is a type of GO:0016753 Sources: EC:2.3.1.103, RHEA:22664